{
  "gene_symbol": "VCX3B",
  "term_id": "UNKNOWN:0001",
  "gene_name": "Variable charge X-linked protein 3B",
  "term_label": "Unknown molecular function",
  "gene": "UniProtKB:Q9H321"
}